{
  "gene_symbol": "DDX3Y",
  "term_id": "GO:0007276",
  "gene": "UniProtKB:O15523",
  "gene_name": "ATP-dependent RNA helicase DDX3Y",
  "term_label": "gamete generation"
}